{
  "term_label": "adherens junction",
  "gene": "UniProtKB:Q9Y446",
  "term_id": "GO:0005912",
  "gene_name": "Plakophilin-3",
  "gene_symbol": "PKP3"
}